{
  "term_label": "extracellular space",
  "gene": "UniProtKB:Q8IWL2",
  "gene_symbol": "SFTPA1",
  "term_id": "GO:0005615",
  "gene_name": "Pulmonary surfactant-associated protein A1"
}